{
  "gene": "UniProtKB:Q3MJ40",
  "term_label": "Unknown cellular component",
  "term_id": "UNKNOWN:0003",
  "gene_name": "Putative coiled-coil domain-containing protein 144B",
  "gene_symbol": "CCDC144BP"
}